{
  "gene_symbol": "KBTBD6",
  "term_id": "GO:0035020",
  "gene_name": "Kelch repeat and BTB domain-containing protein 6",
  "term_label": "regulation of Rac protein signal transduction",
  "gene": "UniProtKB:Q86V97"
}